protocatechuate 3,4-dioxygenase activity [GO:0018578] (molecular function) Relationships: is a type of oxidoreductase activity, acting on single donors with incorporation of molecular oxygen, incorporation of two atoms of oxygen [GO:0016702] Also known as: protocatechuate oxygenase activity, protocatechuate:oxygen 3,4-oxidoreductase (decyclizing), protocatechuic 3,4-dioxygenase activity, protocatechuic 3,4-oxygenase activity, protocatechuic acid oxidase activity Sources: EC:1.13.11.3 Definition: Catalysis of the reaction: 3,4-dihydroxybenzoate + O2 = 3-carboxy-cis,cis-muconate.